{
  "term_id": "GO:0016485",
  "gene": "UniProtKB:Q66K79",
  "gene_symbol": "CPZ",
  "gene_name": "Carboxypeptidase Z",
  "term_label": "protein processing"
}